{
  "gene_symbol": "OAF",
  "gene_name": "Out at first protein homolog",
  "term_id": "UNKNOWN:0002",
  "gene": "UniProtKB:Q86UD1",
  "term_label": "Unknown biological process"
}